{
  "term_label": "DNA-binding transcription factor activity, RNA polymerase II-specific",
  "gene": "UniProtKB:Q147U1",
  "gene_symbol": "ZNF846",
  "gene_name": "Zinc finger protein 846",
  "term_id": "GO:0000981"
}